{
  "gene_symbol": "HSD17B10",
  "gene": "UniProtKB:Q99714",
  "gene_name": "3-hydroxyacyl-CoA dehydrogenase type-2",
  "term_label": "fatty acid metabolic process",
  "term_id": "GO:0006631"
}